{
  "term_id": "GO:0043066",
  "term_label": "negative regulation of apoptotic process",
  "gene_symbol": "FKBP8",
  "gene_name": "Peptidyl-prolyl cis-trans isomerase FKBP8",
  "gene": "UniProtKB:Q14318"
}